{
  "term_id": "GO:1904294",
  "term_label": "positive regulation of ERAD pathway",
  "gene_name": "Ataxin-3-like protein",
  "gene": "UniProtKB:Q9H3M9",
  "gene_symbol": "ATXN3L"
}